{
  "term_id": "GO:0070181",
  "gene": "UniProtKB:Q9BRU9",
  "term_label": "small ribosomal subunit rRNA binding",
  "gene_name": "rRNA-processing protein UTP23 homolog",
  "gene_symbol": "UTP23"
}